{
  "gene": "UniProtKB:P17540",
  "gene_name": "Creatine kinase S-type, mitochondrial",
  "gene_symbol": "CKMT2",
  "term_label": "mitochondrion",
  "term_id": "GO:0005739"
}